{
  "gene": "UniProtKB:A0A0A0MS06",
  "term_label": "plasma membrane",
  "term_id": "GO:0005886",
  "gene_symbol": "TRBV23-1",
  "gene_name": "Probable non-functional T cell receptor beta variable 23-1"
}